{
  "gene_symbol": "UEVLD",
  "term_id": "GO:0043130",
  "gene": "UniProtKB:Q8IX04",
  "gene_name": "Ubiquitin-conjugating enzyme E2 variant 3",
  "term_label": "ubiquitin binding"
}